{
  "gene_symbol": "NUTM2F",
  "gene_name": "NUT family member 2F",
  "term_id": "UNKNOWN:0002",
  "term_label": "Unknown biological process",
  "gene": "UniProtKB:A1L443"
}